{
  "term_label": "protein serine/threonine kinase activity",
  "gene": "UniProtKB:Q9NSY1",
  "term_id": "GO:0004674",
  "gene_symbol": "BMP2K",
  "gene_name": "BMP-2-inducible protein kinase"
}